{
  "term_id": "GO:0033173",
  "gene_name": "Calcineurin subunit B type 1",
  "term_label": "calcineurin-NFAT signaling cascade",
  "gene_symbol": "PPP3R1",
  "gene": "UniProtKB:P63098"
}